lipopolysaccharide binding [GO:0001530] (molecular function) Also known as: endotoxin binding, LPS binding References: PMID:11079463 Relationships: is a type of lipid binding [GO:0008289]; is a type of carbohydrate derivative binding [GO:0097367] Definition: Binding to a lipopolysaccharide.